{
  "term_id": "GO:0004386",
  "gene_symbol": "DHX16",
  "term_label": "helicase activity",
  "gene": "UniProtKB:O60231",
  "gene_name": "Pre-mRNA-splicing factor ATP-dependent RNA helicase DHX16"
}